{
  "term_label": "Unknown molecular function",
  "gene_name": "Pikachurin",
  "gene_symbol": "EGFLAM",
  "term_id": "UNKNOWN:0001",
  "gene": "UniProtKB:Q63HQ2"
}